{
  "term_id": "GO:0004370",
  "gene_name": "Glycerol kinase 3",
  "term_label": "glycerol kinase activity",
  "gene": "UniProtKB:Q14409",
  "gene_symbol": "GK3"
}